dorsal motor nucleus of vagus nerve formation [GO:0035764] (biological process) Definition: The process that gives rise to the dorsal motor nucleus of the vagus nerve. This process pertains to the initial formation of a structure from unspecified parts. Relationships: is a type of anatomical structure formation involved in morphogenesis [GO:0048646]; is part of dorsal motor nucleus of vagus nerve morphogenesis [GO:0035762] Sources: GOC:dgh